systemic acquired resistance, salicylic acid mediated signaling pathway [GO:0009862] (biological process) Definition: The series of molecular signals mediated by salicylic acid involved in systemic acquired resistance. Sources: GOC:jy Also known as: salicylic acid mediated signaling pathway (systemic acquired resistance), systemic acquired resistance, salicylic acid mediated signalling pathway Relationships: is a type of GO:0009863; BFO_0000050 systemic acquired resistance [GO:0009627] Regulation: negatively regulated by symbiont-mediated suppression of defense-related host salicylic acid-mediated signal transduction pathway [GO:0052003]